{
  "gene_name": "Arf-GAP with GTPase, ANK repeat and PH domain-containing protein 1",
  "term_label": "Unknown cellular component",
  "term_id": "UNKNOWN:0003",
  "gene": "UniProtKB:Q9UPQ3",
  "gene_symbol": "AGAP1"
}